{
  "gene_symbol": "KCNH6",
  "gene": "UniProtKB:Q9H252",
  "term_label": "regulation of ventricular cardiac muscle cell membrane repolarization",
  "gene_name": "Potassium voltage-gated channel subfamily H member 6",
  "term_id": "GO:0060307"
}